{
  "term_id": "GO:0035925",
  "gene_symbol": "ZFP36L1",
  "term_label": "mRNA 3'-UTR AU-rich region binding",
  "gene": "UniProtKB:Q07352",
  "gene_name": "mRNA decay activator protein ZFP36L1"
}